{
  "gene": "UniProtKB:Q13838",
  "term_label": "RNA helicase activity",
  "term_id": "GO:0003724",
  "gene_symbol": "DDX39B",
  "gene_name": "Spliceosome RNA helicase DDX39B"
}